{
  "gene": "UniProtKB:Q8N2Q7",
  "term_id": "UNKNOWN:0001",
  "term_label": "Unknown molecular function",
  "gene_symbol": "NLGN1",
  "gene_name": "Neuroligin-1"
}